{
  "gene": "UniProtKB:Q9BQ87",
  "term_label": "regulation of transcription by RNA polymerase II",
  "term_id": "GO:0006357",
  "gene_name": "F-box-like_WD repeat-containing protein TBL1Y",
  "gene_symbol": "TBL1Y"
}